{
  "gene_name": "Probable imidazolonepropionase",
  "gene_symbol": "AMDHD1",
  "term_label": "L-histidine catabolic process",
  "term_id": "GO:0006548",
  "gene": "UniProtKB:Q96NU7"
}